anaerobic acetylene catabolic process [GO:0019487] (biological process) Relationships: is a type of xenobiotic catabolic process [GO:0042178]; is a type of alkyne catabolic process [GO:0043454] Also known as: anaerobic acetylene breakdown, anaerobic acetylene catabolism, anaerobic acetylene degradation, anaerobic ethyne catabolic process, anaerobic ethyne catabolism Sources: ISBN:0721662544 Definition: The chemical reactions and pathways involving acetylene, a colorless, volatile, explosive gas, that occur in the absence of oxygen.